{
  "gene": "UniProtKB:P05015",
  "term_id": "GO:0005125",
  "gene_symbol": "IFNA16",
  "gene_name": "Interferon alpha-16",
  "term_label": "cytokine activity"
}